{
  "term_label": "endoplasmic reticulum membrane",
  "gene": "UniProtKB:Q6E213",
  "term_id": "GO:0005789",
  "gene_name": "Acyl-CoA wax alcohol acyltransferase 2",
  "gene_symbol": "AWAT2"
}